pericentric heterochromatin organization [GO:0140462] (biological process) References: PMID:26744419 Relationships: is a type of heterochromatin formation [GO:0031507] Definition: The organization of chromatin into heterochromatin at the pericentric region of a chromosome.